thiamine kinase activity [GO:0019165] (molecular function) Definition: Catalysis of the reaction: ATP + thiamine = ADP + 2 H+ + thiamine phosphate. Relationships: is a type of kinase activity [GO:0016301]; is a type of phosphotransferase activity, alcohol group as acceptor [GO:0016773] Sources: EC:2.7.1.89, RHEA:12012 Also known as: ATP:thiamin phosphotransferase activity, ATP:thiamine phosphotransferase activity, thiamin kinase (phosphorylating), thiamin kinase activity, thiamin phosphokinase activity